regulation of brown fat cell proliferation [GO:0070347] (biological process) Subtypes: negative regulation of brown fat cell proliferation [GO:0070348], GO:0070349 Relationships: is_a GO:0070344; regulates brown fat cell proliferation [GO:0070342] Also known as: regulation of brown adipocyte proliferation, regulation of brown adipose cell proliferation Sources: GOC:mah, GOC:sl Definition: Any process that modulates the frequency, rate or extent of brown fat cell proliferation.